{
  "term_id": "GO:0005096",
  "term_label": "GTPase activator activity",
  "gene_name": "Rho GTPase-activating protein 31",
  "gene_symbol": "ARHGAP31",
  "gene": "UniProtKB:Q2M1Z3"
}